{
  "gene_symbol": "KLF3",
  "term_id": "GO:0000978",
  "gene_name": "Krueppel-like factor 3",
  "term_label": "RNA polymerase II cis-regulatory region sequence-specific DNA binding",
  "gene": "UniProtKB:P57682"
}